{
  "term_id": "UNKNOWN:0003",
  "gene_name": "UPF0449 protein C19orf25",
  "term_label": "Unknown cellular component",
  "gene_symbol": "C19orf25",
  "gene": "UniProtKB:Q9UFG5"
}